{
  "gene": "UniProtKB:Q9HBX8",
  "gene_symbol": "LGR6",
  "gene_name": "Leucine-rich repeat-containing G-protein coupled receptor 6",
  "term_label": "negative chemotaxis",
  "term_id": "GO:0050919"
}